{
  "gene_symbol": "CDHR2",
  "gene_name": "Cadherin-related family member 2",
  "gene": "UniProtKB:Q9BYE9",
  "term_id": "GO:0005912",
  "term_label": "adherens junction"
}